{
  "gene_name": "Kinesin-associated protein 3",
  "gene": "UniProtKB:Q92845",
  "term_id": "GO:0035869",
  "term_label": "ciliary transition zone",
  "gene_symbol": "KIFAP3"
}